DNA ligase III-XRCC1 complex [GO:0070421] (cellular component) Definition: A protein complex that contains DNA ligase III and XRCC1, and is involved in base excision repair. Relationships: is a type of nuclear protein-containing complex [GO:0140513]; is a type of catalytic complex [GO:1902494] References: PMID:15141024, PMID:7760816